{
  "gene_symbol": "RADIL",
  "gene": "UniProtKB:Q96JH8",
  "term_label": "substrate adhesion-dependent cell spreading",
  "term_id": "GO:0034446",
  "gene_name": "Ras-associating and dilute domain-containing protein"
}